regulation of peptide antigen transport [GO:1901039] (biological process) Subtypes: negative regulation of peptide antigen transport [GO:1901040], positive regulation of peptide antigen transport [GO:1901041] Definition: Any process that modulates the frequency, rate or extent of peptide antigen transport. Sources: GOC:TermGenie, GOC:bf Relationships: is a type of regulation of antigen processing and presentation of peptide antigen [GO:0002583]; is a type of GO:0090087; regulates GO:0046968